reverse gyrase activity [GO:0160097] (molecular function) Relationships: is a type of DNA topoisomerase activity [GO:0003916] References: PMID:25013168 Definition: Catalysis of a DNA topological transformation by transiently cleaving one DNA strand at a time to allow passage of another strand; changes the linking number by +1 per catalytic cycle, is driven by ATP hydrolysis.